{
  "term_id": "GO:0005737",
  "term_label": "cytoplasm",
  "gene_symbol": "VRK2",
  "gene": "UniProtKB:Q86Y07",
  "gene_name": "Serine_threonine-protein kinase VRK2"
}